negative regulation of centriole-centriole cohesion [GO:1903126] (biological process) References: PMID:24554434 Sources: GOC:TermGenie, GOC:als, GO_REF:0000058 Definition: Any process that stops, prevents or reduces the frequency, rate or extent of centriole-centriole cohesion. Also known as: down regulation of centriole-centriole cohesion, down-regulation of centriole-centriole cohesion, downregulation of centriole-centriole cohesion, inhibition of centriole-centriole cohesion Relationships: is a type of GO:0010948; is a type of regulation of centriole-centriole cohesion [GO:0030997]; negatively regulates centriole-centriole cohesion [GO:0010457]